phosphocreatine catabolic process [GO:0046315] (biological process) Sources: GOC:ai Definition: The chemical reactions and pathways resulting in the breakdown of phosphocreatine, a phosphagen of creatine which is synthesized and broken down by creatine phosphokinase. Also known as: phosphocreatine breakdown, phosphocreatine catabolism, phosphocreatine degradation Relationships: is_a phosphocreatine metabolic process [GO:0006603]; is a type of GO:0042397